{
  "gene_symbol": "TEKT4",
  "term_id": "GO:0060271",
  "gene_name": "Tektin-4",
  "gene": "UniProtKB:Q8WW24",
  "term_label": "cilium assembly"
}